{
  "gene_symbol": "CACNA2D4",
  "gene": "UniProtKB:Q7Z3S7",
  "term_label": "Unknown biological process",
  "term_id": "UNKNOWN:0002",
  "gene_name": "Voltage-dependent calcium channel subunit alpha-2_delta-4"
}